{
  "gene": "UniProtKB:P30874",
  "term_id": "GO:0004994",
  "term_label": "somatostatin receptor activity",
  "gene_name": "Somatostatin receptor type 2",
  "gene_symbol": "SSTR2"
}